icosanoid biosynthetic process [GO:0046456] (biological process) Sources: ISBN:0198506732 Subtypes: leukotriene biosynthetic process [GO:0019370], prostanoid biosynthetic process [GO:0046457] Also known as: eicosanoid biosynthesis, eicosanoid biosynthetic process, eoxin biosynthesis, eoxin synthesis, icosanoid anabolism, icosanoid biosynthesis, icosanoid formation, icosanoid synthesis Relationships: is a type of icosanoid metabolic process [GO:0006690]; is a type of carboxylic acid biosynthetic process [GO:0046394] Definition: The chemical reactions and pathways resulting in the formation of icosanoids, any of a group of C20 polyunsaturated fatty acids.